{
  "gene_symbol": "RTCA",
  "term_label": "nucleus",
  "gene_name": "RNA 3'-terminal phosphate cyclase",
  "term_id": "GO:0005634",
  "gene": "UniProtKB:O00442"
}